phosphatase regulator activity [GO:0019208] (molecular function) Relationships: is a type of enzyme regulator activity [GO:0030234]; has part phosphatase binding [GO:0019902]; regulates GO:0016791 Subtypes: phosphatase activator activity [GO:0019211], GO:0019212, GO:0019888 Definition: Binds to and modulates the activity of a phosphatase, an enzyme which catalyzes of the removal of a phosphate group from a substrate molecule. Sources: GOC:ai